{
  "gene_name": "Bromodomain testis-specific protein",
  "gene_symbol": "BRDT",
  "gene": "UniProtKB:Q58F21",
  "term_id": "GO:0042393",
  "term_label": "histone binding"
}